{
  "term_id": "UNKNOWN:0001",
  "term_label": "Unknown molecular function",
  "gene_symbol": "PAEP",
  "gene": "UniProtKB:P09466",
  "gene_name": "Glycodelin"
}